{
  "term_label": "odorant binding",
  "gene": "UniProtKB:Q8NGG2",
  "gene_symbol": "OR5T2",
  "gene_name": "Olfactory receptor 5T2",
  "term_id": "GO:0005549"
}